{
  "gene": "UniProtKB:Q9UL12",
  "term_label": "sarcosine dehydrogenase activity",
  "gene_symbol": "SARDH",
  "gene_name": "Sarcosine dehydrogenase, mitochondrial",
  "term_id": "GO:0008480"
}